mesonephric mesenchyme development [GO:0061219] (biological process) Relationships: is a type of kidney mesenchyme development [GO:0072074]; is part of mesonephros development [GO:0001823] Definition: The biological process whose specific outcome is the progression of a mesonephric mesenchyme from an initial condition to its mature state. This process begins with the formation of mesonephric mesenchyme and ends with the mature structure. Mesonephric mesenchyme is the tissue made up of loosely connected mesenchymal cells in the mesonephros. Sources: GOC:mtg_kidney_jan10